efferent axon development in a lateral line nerve [GO:0048894] (biological process) Subtypes: efferent axon development in anterior lateral line nerve [GO:0048911], efferent axon development in posterior lateral line nerve [GO:0048929] Definition: The process whose specific outcome is the progression of an efferent axon in a lateral line nerve over time from its formation to the mature structure. This process includes axonogenesis and pathfinding of the efferent axons in any lateral line nerve. Relationships: is a type of central nervous system neuron axonogenesis [GO:0021955]; is part of lateral line nerve development [GO:0048892] References: PMID:15832385